{
  "gene_name": "Guanosine-3',5'-bis(diphosphate) 3'-pyrophosphohydrolase MESH1",
  "term_id": "UNKNOWN:0002",
  "term_label": "Unknown biological process",
  "gene_symbol": "HDDC3",
  "gene": "UniProtKB:Q8N4P3"
}